regulation of xylan catabolic process [GO:2001000] (biological process) Also known as: regulation of xylan breakdown, regulation of xylan catabolism, regulation of xylan degradation Relationships: is a type of regulation of hemicellulose catabolic process [GO:2000988]; regulates xylan catabolic process [GO:0045493] Subtypes: regulation of glucuronoxylan catabolic process [GO:2000915], regulation of arabinoxylan-containing compound catabolic process [GO:2000921], negative regulation of xylan catabolic process [GO:2001001], positive regulation of xylan catabolic process [GO:2001002] Sources: GOC:mengo_curators Definition: Any process that modulates the frequency, rate or extent of xylan catabolic process.